cholesterol transport [GO:0030301] (biological process) Sources: GOC:mah, ISBN:0198506732 Relationships: is a type of sterol transport [GO:0015918] Regulation: regulated by GO:0032374; negatively regulated by negative regulation of cholesterol transport [GO:0032375]; positively regulated by positive regulation of cholesterol transport [GO:0032376] Definition: The directed movement of cholesterol, cholest-5-en-3-beta-ol, into, out of or within a cell, or between cells, by means of some agent such as a transporter or pore. Subtypes: cholesterol transport involved in cholesterol storage [GO:0010879], intracellular cholesterol transport [GO:0032367], GO:0033344, reverse cholesterol transport [GO:0043691], GO:0070508